{
  "gene_name": "Nuclear receptor subfamily 1 group I member 2",
  "gene_symbol": "NR1I2",
  "gene": "UniProtKB:O75469",
  "term_id": "GO:0030522",
  "term_label": "intracellular receptor signaling pathway"
}